{
  "gene_symbol": "ZDHHC11",
  "term_label": "protein-cysteine S-palmitoyltransferase activity",
  "gene": "UniProtKB:Q9H8X9",
  "term_id": "GO:0019706",
  "gene_name": "Palmitoyltransferase ZDHHC11"
}